{
  "gene": "UniProtKB:Q9H6R6",
  "gene_symbol": "ZDHHC6",
  "gene_name": "Palmitoyltransferase ZDHHC6",
  "term_label": "Golgi apparatus",
  "term_id": "GO:0005794"
}